{
  "gene_name": "FOXL2 neighbor protein",
  "gene_symbol": "FOXL2NB",
  "term_label": "Unknown biological process",
  "gene": "UniProtKB:Q6ZUU3",
  "term_id": "UNKNOWN:0002"
}